{
  "gene_name": "PR domain zinc finger protein 4",
  "gene_symbol": "PRDM4",
  "term_label": "nucleus",
  "term_id": "GO:0005634",
  "gene": "UniProtKB:Q9UKN5"
}